acetoin-ribose-5-phosphate transaldolase activity [GO:0047156] (molecular function) Definition: Catalysis of the reaction: D-ribose 5-phosphate + acetoin = 1-deoxy-D-altro-heptulose 7-phosphate + acetaldehyde. Relationships: is a type of transketolase or transaldolase activity [GO:0016744] Sources: RHEA:21504 Also known as: 1-deoxy-D-altro-heptulose-7-phosphate synthase activity, 1-deoxy-D-altro-heptulose-7-phosphate synthetase activity, 3-hydroxybutan-2-one:D-ribose-5-phosphate aldehydetransferase activity, 3-hydroxybutan-3-one:D-ribose-5-phosphate aldehydetransferase activity